{
  "term_id": "GO:0005834",
  "term_label": "heterotrimeric G-protein complex",
  "gene_name": "Guanine nucleotide-binding protein G(I)_G(S)_G(O) subunit gamma-8",
  "gene": "UniProtKB:Q9UK08",
  "gene_symbol": "GNG8"
}